{
  "gene_name": "E3 ubiquitin-protein ligase RNF8",
  "term_label": "site of double-strand break",
  "gene": "UniProtKB:O76064",
  "term_id": "GO:0035861",
  "gene_symbol": "RNF8"
}